{
  "term_label": "histone H4K20 methyltransferase activity",
  "gene_symbol": "KMT5A",
  "gene": "UniProtKB:Q9NQR1",
  "term_id": "GO:0042799",
  "gene_name": "N-lysine methyltransferase KMT5A"
}